{
  "gene": "UniProtKB:Q4G0G2",
  "term_label": "Unknown molecular function",
  "gene_symbol": "H1-10-AS1",
  "term_id": "UNKNOWN:0001",
  "gene_name": "Putative uncharacterized protein H1-10-AS1"
}